{
  "term_label": "heparan sulfate proteoglycan biosynthetic process",
  "gene_symbol": "GLCE",
  "gene_name": "D-glucuronyl C5-epimerase",
  "term_id": "GO:0015012",
  "gene": "UniProtKB:O94923"
}